protein insertion into membrane [GO:0051205] (biological process) Also known as: integral membrane protein localization, integral membrane protein positioning, membrane protein localization, membrane protein positioning, protein-membrane insertion Subtypes: GO:0045048, protein insertion into mitochondrial membrane [GO:0051204], protein insertion into membrane raft [GO:0071210], protein insertion into plasma membrane [GO:0098737] Relationships: is a type of GO:0090150; is part of GO:0008104; is part of GO:0061024 Sources: GOC:ai Definition: The process that results in the incorporation of a protein into a biological membrane. Incorporation in this context means having some part or covalently attached group that is inserted into the the hydrophobic region of one or both bilayers.